{
  "gene": "UniProtKB:Q93009",
  "term_label": "regulation of protein stability",
  "gene_symbol": "USP7",
  "term_id": "GO:0031647",
  "gene_name": "Ubiquitin carboxyl-terminal hydrolase 7"
}